lipopolysaccharide-1,5-galactosyltransferase activity [GO:0035496] (molecular function) Definition: Catalysis of the reaction: UDP-galactose + lipopolysaccharide = UDP + 1,5 alpha-D-galactosyl-lipopolysaccharide. References: PMID:11304545 Also known as: LPS-1,5-galactosyltransferase activity, UDP-D-galactose:(glucosyl)lipopolysaccharide-1,5-D-galactosyltransferase Relationships: is a type of UDP-galactosyltransferase activity [GO:0035250]